menadiol geranylgeranyltransferase activity [GO:0120566] (molecular function) Relationships: is a type of prenyltransferase activity [GO:0004659] Definition: Catalysis of the reaction: menadiol + (2E,6E,10E)-geranylgeranyl diphosphate = menaquinol-4 + diphosphate. References: PMID:20953171 Sources: RHEA:74083